{
  "gene": "UniProtKB:Q9NS69",
  "term_label": "protein import into mitochondrial matrix",
  "gene_symbol": "TOMM22",
  "term_id": "GO:0030150",
  "gene_name": "Mitochondrial import receptor subunit TOM22 homolog"
}